{
  "gene_name": "Cytokine-inducible SH2-containing protein",
  "term_label": "Unknown cellular component",
  "term_id": "UNKNOWN:0003",
  "gene_symbol": "CISH",
  "gene": "UniProtKB:Q9NSE2"
}